{
  "gene_symbol": "CDC73",
  "term_label": "RNA polymerase II complex binding",
  "gene": "UniProtKB:Q6P1J9",
  "gene_name": "Parafibromin",
  "term_id": "GO:0000993"
}